{
  "gene": "UniProtKB:Q8IXS6",
  "term_label": "Unknown molecular function",
  "gene_symbol": "PALM2",
  "gene_name": "Paralemmin-2",
  "term_id": "UNKNOWN:0001"
}